{
  "term_id": "GO:0006273",
  "gene_name": "DNA ligase 1",
  "gene": "UniProtKB:P18858",
  "gene_symbol": "LIG1",
  "term_label": "lagging strand elongation"
}